{
  "term_id": "UNKNOWN:0003",
  "term_label": "Unknown cellular component",
  "gene_symbol": "C1orf100",
  "gene_name": "Uncharacterized protein C1orf100",
  "gene": "UniProtKB:Q5SVJ3"
}